long-chain-alcohol dehydrogenase activity [GO:0050060] (molecular function) Also known as: fatty alcohol oxidoreductase activity, long-chain alcohol dehydrogenase activity, long-chain-alcohol:NAD+ oxidoreductase activity Relationships: is a type of GO:0016616 Definition: Catalysis of the reaction: a long-chain alcohol + 2 NAD+ + H2O = a long-chain carboxylate + 2 NADH. Sources: EC:1.1.1.192, MetaCyc:LONG-CHAIN-ALCOHOL-DEHYDROGENASE-RXN